{
  "gene_symbol": "FCHSD1",
  "gene": "UniProtKB:Q86WN1",
  "term_id": "GO:0055037",
  "term_label": "recycling endosome",
  "gene_name": "F-BAR and double SH3 domains protein 1"
}